{
  "term_id": "GO:0006354",
  "gene_symbol": "AFF4",
  "gene_name": "AF4_FMR2 family member 4",
  "term_label": "DNA-templated transcription elongation",
  "gene": "UniProtKB:Q9UHB7"
}